{
  "term_id": "GO:0004683",
  "gene": "UniProtKB:Q16566",
  "term_label": "calcium/calmodulin-dependent protein kinase activity",
  "gene_symbol": "CAMK4",
  "gene_name": "Calcium_calmodulin-dependent protein kinase type IV"
}